{
  "term_label": "Unknown cellular component",
  "gene": "UniProtKB:Q5BKX5",
  "gene_symbol": "ACTMAP",
  "gene_name": "Actin maturation protease",
  "term_id": "UNKNOWN:0003"
}